{
  "gene": "UniProtKB:A8MVA2",
  "gene_symbol": "KRTAP9-6",
  "term_id": "UNKNOWN:0002",
  "term_label": "Unknown biological process",
  "gene_name": "Keratin-associated protein 9-6"
}